{
  "term_label": "extracellular matrix",
  "gene": "UniProtKB:P07996",
  "gene_name": "Thrombospondin-1",
  "term_id": "GO:0031012",
  "gene_symbol": "THBS1"
}